{
  "gene_symbol": "UNC5C",
  "term_label": "netrin receptor activity",
  "term_id": "GO:0005042",
  "gene_name": "Netrin receptor UNC5C",
  "gene": "UniProtKB:O95185"
}